{
  "gene_name": "GTPase Era, mitochondrial",
  "gene_symbol": "ERAL1",
  "term_id": "GO:0000028",
  "gene": "UniProtKB:O75616",
  "term_label": "ribosomal small subunit assembly"
}